{
  "gene_name": "B-cell lymphoma 6 protein",
  "gene": "UniProtKB:P41182",
  "gene_symbol": "BCL6",
  "term_label": "regulation of cytokine production",
  "term_id": "GO:0001817"
}